{
  "gene_name": "Jerky protein homolog-like",
  "term_id": "GO:0003677",
  "term_label": "DNA binding",
  "gene": "UniProtKB:Q9Y4A0",
  "gene_symbol": "JRKL"
}